sulfonylurea receptor activity [GO:0008281] (molecular function) Definition: Combining with sulfonylurea, and transmitting the signal from one side of the membrane to the other to initiate a change in cell activity. Sources: GOC:ai, GOC:signaling Relationships: is a type of GO:0004888 Also known as: sulphonylurea receptor activity Note: Note that this term represents an activity and not a gene product. Consider also annotating to the molecular function term 'potassium channel activity ; GO:0005267'.